regulation of response to water deprivation [GO:2000070] (biological process) Relationships: is_a regulation of response to stress [GO:0080134]; regulates response to water deprivation [GO:0009414] Also known as: regulation of response to dehydration, regulation of response to drought, regulation of response to thirst, regulation of drought tolerance Subtypes: GO:0080148, positive regulation of response to water deprivation [GO:1902584] Sources: GOC:obol Definition: Any process that modulates the frequency, rate or extent of response to water deprivation.